second spliceosomal transesterification activity [GO:0000386] (molecular function) Also known as: 3'-splice site cleavage, exon ligation, lariat formation, 5'-splice site cleavage References: PMID:19239890 Sources: GOC:krc, ISBN:0879695897 Relationships: is a type of GO:0140098; is part of GO:0000375 Definition: Catalysis of the second transesterification reaction of spliceosomal mRNA splicing. Ligation of the two exons occurs via a transesterification reaction where the free 3'-hydroxyl group of the 5' exon is the nucleophile attacking the 3' splice site. Non-expressed sequences are now detached from the exons. In cis splicing, the intron is in a lariat structure.